L-threonine catabolic process to D-lactate [GO:0019517] (biological process) Also known as: L-threonine catabolic process to (R)-lactate, threonine catabolic process to D-lactate, L-threonine breakdown to D-lactate, L-threonine catabolic process to methylglyoxal, L-threonine catabolism to D-lactate, L-threonine degradation to D-lactate, L-threonine catabolic process to pyruvate Sources: GOC:bf, GOC:jl, MetaCyc:THRDLCTCAT-PWY Definition: The chemical reactions and pathways resulting in the breakdown of L- threonine (the L-enantiomer of 2-amino-3-hydroxybutyric acid) to form the compound methylglyoxal, which is subsequently converted to D-lactate. Relationships: is_a lactate metabolic process [GO:0006089]; is a type of L-threonine catabolic process [GO:0006567]